detection of nodal flow [GO:0003127] (biological process) Definition: The series of events by which an endogenous stimulus is received by a cilium on a cell and converted to a molecular signal contributing to left/right asymmetry. Sources: GOC:mtg_heart Relationships: is a type of GO:0071495; is part of determination of left/right symmetry [GO:0007368]